endopeptidase activator activity [GO:0061133] (molecular function) Definition: Binds to and increases the activity of an endopeptidase. Sources: GOC:dph, GOC:tb Relationships: is_a peptidase activator activity [GO:0016504]; is_a endopeptidase regulator activity [GO:0061135]; positively regulates endopeptidase activity [GO:0004175] Subtypes: cysteine-type endopeptidase activator activity [GO:0140608]